{
  "term_id": "GO:0010165",
  "gene_symbol": "XRCC4",
  "term_label": "response to X-ray",
  "gene_name": "DNA repair protein XRCC4",
  "gene": "UniProtKB:Q13426"
}